purine nucleotide transport [GO:0015865] (biological process) Definition: The directed movement of a purine nucleotide, any compound consisting of a purine nucleoside esterified with (ortho)phosphate, into, out of or within a cell. Sources: GOC:ai Relationships: is_a nucleotide transport [GO:0006862] Subtypes: GO:0001408, GO:0015868, adenine nucleotide transport [GO:0051503]